{
  "gene_symbol": "UGT1A5",
  "term_id": "GO:0008194",
  "term_label": "UDP-glycosyltransferase activity",
  "gene_name": "UDP-glucuronosyltransferase 1A5",
  "gene": "UniProtKB:P35504"
}